{
  "term_id": "GO:0005829",
  "gene": "UniProtKB:O00628",
  "term_label": "cytosol",
  "gene_name": "Peroxisomal targeting signal 2 receptor",
  "gene_symbol": "PEX7"
}